{
  "gene_symbol": "GCLM",
  "gene_name": "Glutamate--cysteine ligase regulatory subunit",
  "term_label": "glutamate-cysteine ligase catalytic subunit binding",
  "gene": "UniProtKB:P48507",
  "term_id": "GO:0035226"
}